{
  "gene_name": "Transcription elongation factor SPT5",
  "gene_symbol": "SUPT5H",
  "term_label": "transcription elongation by RNA polymerase II",
  "term_id": "GO:0006368",
  "gene": "UniProtKB:O00267"
}